{
  "gene_name": "NADH-ubiquinone oxidoreductase chain 1",
  "term_label": "aerobic respiration",
  "term_id": "GO:0009060",
  "gene_symbol": "MT-ND1",
  "gene": "UniProtKB:P03886"
}